regulation of endothelial cell differentiation [GO:0045601] (biological process) Subtypes: GO:0045602, positive regulation of endothelial cell differentiation [GO:0045603], regulation of blood vessel endothelial cell differentiation [GO:0110057], regulation of endothelial cell development [GO:1901550] Sources: GOC:go_curators Definition: Any process that modulates the frequency, rate or extent of endothelial cell differentiation. Relationships: is a type of GO:0030856; regulates endothelial cell differentiation [GO:0045446]